{
  "term_id": "GO:0004861",
  "term_label": "cyclin-dependent protein serine/threonine kinase inhibitor activity",
  "gene_symbol": "CDKN1B",
  "gene_name": "Cyclin-dependent kinase inhibitor 1B",
  "gene": "UniProtKB:P46527"
}